{
  "gene_symbol": "SLC22A8",
  "gene_name": "Organic anion transporter 3",
  "term_id": "GO:0015711",
  "term_label": "organic anion transport",
  "gene": "UniProtKB:Q8TCC7"
}